{
  "gene_name": "Ubiquitin carboxyl-terminal hydrolase 17-like protein 12",
  "gene_symbol": "USP17L12",
  "gene": "UniProtKB:C9JPN9",
  "term_id": "GO:0042981",
  "term_label": "regulation of apoptotic process"
}